depurination [GO:0045007] (biological process) Definition: The disruption of the bond between the sugar in the backbone and the A or G base, causing the base to be removed and leaving a depurinated sugar. Sources: GOC:ai Relationships: is a type of base-excision repair, AP site formation [GO:0006285]; is a type of GO:0006304